lumenal side of early endosome membrane [GO:0098550] (cellular component) Relationships: is a type of GO:0098565; is part of early endosome membrane [GO:0031901] Definition: The side (leaflet) of the early endosome membrane that faces the lumen. Sources: GOC:lr Also known as: internal leaflet of early endosome membrane, internal side of early endosome membrane